{
  "gene_name": "Cell division control protein 42 homolog",
  "term_id": "GO:0030010",
  "term_label": "establishment of cell polarity",
  "gene": "UniProtKB:P60953",
  "gene_symbol": "CDC42"
}